{
  "term_id": "GO:0030246",
  "gene_symbol": "CLEC6A",
  "term_label": "carbohydrate binding",
  "gene": "UniProtKB:Q6EIG7",
  "gene_name": "C-type lectin domain family 6 member A"
}